{
  "term_label": "cytosol",
  "term_id": "GO:0005829",
  "gene_symbol": "GNMT",
  "gene": "UniProtKB:Q14749",
  "gene_name": "Glycine N-methyltransferase"
}